{
  "gene": "UniProtKB:P78549",
  "term_label": "DNA-(apurinic or apyrimidinic site) endonuclease activity",
  "gene_symbol": "NTHL1",
  "gene_name": "Endonuclease III-like protein 1",
  "term_id": "GO:0003906"
}